D-aspartate ligase activity [GO:0034025] (molecular function) Sources: EC:6.3.1.12 Relationships: is a type of acid-ammonia (or amide) ligase activity [GO:0016880] Also known as: D-aspartate:[beta-GlcNAc-(1->4)-Mur2Ac(oyl-L-Ala-gamma-D-Glu-L-Lys-D-Ala-D-Ala)]n ligase (ADP-forming) activity, D-aspartic acid-activating enzyme, UDP-MurNAc-pentapeptide:D-aspartate ligase activity, aslfm Definition: Catalysis of the reaction: ATP + D-aspartate + [beta-GlcNAc-(1->4)-Mur2Ac(oyl-L-Ala-gamma-D-Glu-L-Lys-D-Ala-D-Ala)]n = [beta-GlcNAc-(1->4)-Mur2Ac(oyl-L-Ala-gamma-D-Glu-6-N-(beta-D-Asp)-L-Lys-D-Ala-D-Ala)]n + ADP + phosphate.